regulation of antipodal cell differentiation [GO:0045688] (biological process) Definition: Any process that modulates the frequency, rate or extent of antipodal cell differentiation. Relationships: is a type of regulation of cell differentiation [GO:0045595]; regulates antipodal cell differentiation [GO:0009557] Subtypes: GO:0045689, positive regulation of antipodal cell differentiation [GO:0045690] Sources: GOC:go_curators, GOC:mtg_plant